{
  "term_label": "central nervous system myelin maintenance",
  "gene_name": "Myelin regulatory factor",
  "gene_symbol": "MYRF",
  "gene": "UniProtKB:Q9Y2G1",
  "term_id": "GO:0032286"
}